ketoreductase activity [GO:0045703] (molecular function) Definition: Catalysis of the reduction of a ketone group to form the corresponding alcohol. Subtypes: norsolorinic acid ketoreductase activity [GO:0140393] Relationships: is a type of oxidoreductase activity, acting on CH-OH group of donors [GO:0016614] Sources: GOC:curators